{
  "term_label": "inflammatory response",
  "gene": "UniProtKB:Q9UNI1",
  "gene_name": "Chymotrypsin-like elastase family member 1",
  "term_id": "GO:0006954",
  "gene_symbol": "CELA1"
}